RNA ligase (GTP) activity [GO:0170057] (molecular function) Relationships: is a type of RNA ligase activity [GO:0008452] References: PMID:21311021 Sources: EC:6.5.1.8 Definition: Catalysis of the joining of an RNA with 3'-phosphate or 2',3'-cyclic-phosphate ends to an RNA with 5'-hydroxy ends according to either (i) a 3'-end 3'-phospho-ribonucleotide-RNA + a 5'-end dephospho-ribonucleoside-RNA + GTP = a ribonucleotidyl-ribonucleotide-RNA + diphosphate + GMP; or (ii) a 3'-end 2',3'-cyclophospho-ribonucleotide-RNA + a 5'-end dephospho-ribonucleoside-RNA + GTP + H2O = a ribonucleotidyl-ribonucleotide-RNA + diphosphate + GMP + H+. Also known as: 3'-phosphate/5'-hydroxy nucleic acid ligase activity